{
  "term_id": "GO:0005819",
  "term_label": "spindle",
  "gene_symbol": "EMD",
  "gene": "UniProtKB:P50402",
  "gene_name": "Emerin"
}